{
  "term_label": "Unknown molecular function",
  "gene_symbol": "CCDC92B",
  "gene": "UniProtKB:A0A8I5KY20",
  "gene_name": "Coiled-coil domain containing 92B",
  "term_id": "UNKNOWN:0001"
}